{
  "gene_symbol": "SFTPA1",
  "gene_name": "Pulmonary surfactant-associated protein A1",
  "term_label": "multivesicular body",
  "gene": "UniProtKB:Q8IWL2",
  "term_id": "GO:0005771"
}